{
  "gene_name": "Protein kinase C-binding protein NELL2",
  "gene_symbol": "NELL2",
  "term_label": "extracellular space",
  "gene": "UniProtKB:Q99435",
  "term_id": "GO:0005615"
}